{
  "term_label": "maturation of SSU-rRNA",
  "gene": "UniProtKB:Q9UI30",
  "term_id": "GO:0030490",
  "gene_name": "Multifunctional methyltransferase subunit TRM112-like protein",
  "gene_symbol": "TRMT112"
}